octopamine receptor activity [GO:0004989] (molecular function) Relationships: is a type of G protein-coupled amine receptor activity [GO:0008227] Definition: Combining with the biogenic amine octopamine to initiate a change in cell activity. Octopamine is found in both vertebrates and invertebrates and can have properties both of a hormone and a neurotransmitter and acts as an adrenergic agonist. Sources: GOC:ai